positive regulation of asperthecin biosynthetic process [GO:1900381] (biological process) Sources: GOC:TermGenie, GOC:di Also known as: activation of asperthecin biosynthesis, activation of asperthecin formation, activation of asperthecin synthesis, positive regulation of asperthecin biosynthesis, positive regulation of asperthecin formation, positive regulation of asperthecin synthesis, up regulation of asperthecin biosynthesis, up regulation of asperthecin biosynthetic process, up regulation of asperthecin formation, up regulation of asperthecin synthesis, up-regulation of asperthecin biosynthesis, up-regulation of asperthecin biosynthetic process, up-regulation of asperthecin formation, up-regulation of asperthecin synthesis, upregulation of asperthecin biosynthesis, upregulation of asperthecin biosynthetic process, upregulation of asperthecin formation, upregulation of asperthecin synthesis, activation of asperthecin biosynthetic process Relationships: is a type of GO:0062013; is a type of positive regulation of secondary metabolite biosynthetic process [GO:1900378]; is a type of regulation of asperthecin biosynthetic process [GO:1900379]; positively regulates GO:0036184 Definition: Any process that activates or increases the frequency, rate or extent of asperthecin biosynthetic process.